{
  "gene": "UniProtKB:Q9UMS5",
  "term_id": "UNKNOWN:0002",
  "gene_symbol": "PHTF1",
  "gene_name": "Protein PHTF1",
  "term_label": "Unknown biological process"
}